{
  "gene_symbol": "ST3GAL4",
  "gene_name": "CMP-N-acetylneuraminate-beta-galactosamide-alpha-2,3-sialyltransferase 4",
  "term_label": "beta-D-galactosyl-(1->3)-N-acetyl-beta-D-galactosaminide alpha-2,3- sialyltransferase",
  "gene": "UniProtKB:Q11206",
  "term_id": "GO:0047288"
}